positive regulation of epinephrine secretion [GO:0032812] (biological process) Sources: GOC:vk Also known as: positive regulation of adrenaline secretion, up regulation of epinephrine secretion, up-regulation of epinephrine secretion, upregulation of epinephrine secretion, activation of epinephrine secretion, stimulation of epinephrine secretion Relationships: is a type of regulation of epinephrine secretion [GO:0014060]; is a type of GO:0033605; positively regulates epinephrine secretion [GO:0048242] Definition: Any process that activates or increases the frequency, rate or extent of the regulated release of epinephrine.